{
  "term_label": "structural constituent of chromatin",
  "gene_name": "Histone H2B type 1-N",
  "gene": "UniProtKB:Q99877",
  "gene_symbol": "H2BC15",
  "term_id": "GO:0030527"
}